{
  "term_label": "plasma membrane",
  "gene_name": "Ceramide kinase-like protein",
  "gene": "UniProtKB:Q49MI3",
  "term_id": "GO:0005886",
  "gene_symbol": "CERKL"
}